{
  "gene_name": "Matrix metalloproteinase-14",
  "gene_symbol": "MMP14",
  "term_label": "metalloendopeptidase activity",
  "gene": "UniProtKB:P50281",
  "term_id": "GO:0004222"
}